negative regulation of DNA damage checkpoint [GO:2000002] (biological process) Subtypes: GO:1904290 Relationships: is a type of negative regulation of cell cycle checkpoint [GO:1901977]; is a type of regulation of DNA damage checkpoint [GO:2000001]; negatively regulates DNA damage checkpoint signaling [GO:0000077] Also known as: negative regulation of DNA damage response, signal transduction resulting in cell cycle arrest Definition: Any process that stops, prevents, or reduces the frequency, rate or extent of a DNA damage checkpoint. Sources: GOC:BHF, GOC:obol